steroid hormone receptor signaling pathway [GO:0043401] (biological process) Subtypes: GO:0009742, nuclear receptor-mediated steroid hormone signaling pathway [GO:0030518] References: PMID:12606724 Definition: The series of molecular signals mediated by a steroid hormone binding to a receptor. Relationships: is a type of hormone-mediated signaling pathway [GO:0009755]; is part of cellular response to steroid hormone stimulus [GO:0071383] Also known as: steroid hormone mediated signalling, steroid hormone-mediated signaling pathway